{
  "term_label": "DNA-binding transcription factor activity, RNA polymerase II-specific",
  "gene_name": "Krueppel-like factor 11",
  "gene": "UniProtKB:O14901",
  "term_id": "GO:0000981",
  "gene_symbol": "KLF11"
}